{
  "term_id": "GO:0050804",
  "gene_symbol": "GRIA1",
  "gene": "UniProtKB:P42261",
  "gene_name": "Glutamate receptor 1",
  "term_label": "modulation of chemical synaptic transmission"
}